specific granule [GO:0042581] (cellular component) References: PMID:7334549 Sources: GOC:jl, ISBN:0721662544 Relationships: is a type of secretory granule [GO:0030141] Also known as: secondary granule Definition: Granule with a membranous, tubular internal structure, found primarily in mature neutrophil cells. Most are released into the extracellular fluid. Specific granules contain lactoferrin, lysozyme, vitamin B12 binding protein and elastase.